{
  "term_label": "protein ubiquitination",
  "gene_name": "E3 ubiquitin-protein ligase Praja-1",
  "term_id": "GO:0016567",
  "gene": "UniProtKB:Q8NG27",
  "gene_symbol": "PJA1"
}